{
  "gene_symbol": "LARP1B",
  "term_id": "GO:0005829",
  "gene_name": "La-related protein 1B",
  "gene": "UniProtKB:Q659C4",
  "term_label": "cytosol"
}